{
  "gene": "UniProtKB:P07451",
  "gene_symbol": "CA3",
  "term_id": "GO:0004089",
  "gene_name": "Carbonic anhydrase 3",
  "term_label": "carbonate dehydratase activity"
}